{
  "gene_symbol": "ACO2",
  "term_id": "GO:0051539",
  "gene": "UniProtKB:Q99798",
  "term_label": "4 iron, 4 sulfur cluster binding",
  "gene_name": "Aconitate hydratase, mitochondrial"
}